{
  "gene_name": "GTPase HRas",
  "gene_symbol": "HRAS",
  "term_id": "GO:0008284",
  "gene": "UniProtKB:P01112",
  "term_label": "positive regulation of cell population proliferation"
}